{
  "term_label": "RNA polymerase II cis-regulatory region sequence-specific DNA binding",
  "term_id": "GO:0000978",
  "gene_name": "Zinc finger protein 1 homolog",
  "gene": "UniProtKB:Q6P2D0",
  "gene_symbol": "ZFP1"
}